{
  "gene_symbol": "PRPF31",
  "term_label": "mRNA splicing, via spliceosome",
  "gene": "UniProtKB:Q8WWY3",
  "term_id": "GO:0000398",
  "gene_name": "U4_U6 small nuclear ribonucleoprotein Prp31"
}